{
  "gene": "UniProtKB:Q9NRH1",
  "gene_symbol": "YAE1",
  "term_id": "UNKNOWN:0002",
  "gene_name": "Protein YAE1 homolog",
  "term_label": "Unknown biological process"
}